positive regulation of proteolysis involved in protein catabolic process [GO:1903052] (biological process) Relationships: is a type of positive regulation of proteolysis [GO:0045862]; is a type of regulation of proteolysis involved in protein catabolic process [GO:1903050]; positively regulates proteolysis involved in protein catabolic process [GO:0051603] References: PMID:18307834 Sources: GOC:BHF, GOC:TermGenie, GOC:rl, GO_REF:0000058 Note: overexpression of cathepsin C propeptide significantly increased the degradation of intestinal alkaline phosphatase (IAP) Also known as: positive regulation of peptidolysis involved in cellular protein catabolic process, positive regulation of peptidolysis involved in cellular protein catabolism, positive regulation of proteolysis involved in cellular protein catabolic process, up regulation of peptidolysis involved in cellular protein catabolic process, up regulation of peptidolysis involved in cellular protein catabolism, up regulation of proteolysis involved in cellular protein catabolic process, up-regulation of peptidolysis involved in cellular protein catabolic process, up-regulation of peptidolysis involved in cellular protein catabolism, up-regulation of proteolysis involved in cellular protein catabolic process, upregulation of peptidolysis involved in cellular protein catabolic process, upregulation of peptidolysis involved in cellular protein catabolism, upregulation of proteolysis involved in cellular protein catabolic process, activation of peptidolysis involved in cellular protein catabolic process, activation of peptidolysis involved in cellular protein catabolism, activation of proteolysis involved in cellular protein catabolic process, activation of peptidolysis during cellular protein catabolic process, activation of peptidolysis during cellular protein catabolism, activation of proteolysis during cellular protein catabolic process, activation of proteolysis during cellular protein catabolism, positive regulation of peptidolysis during cellular protein catabolic process, positive regulation of peptidolysis during cellular protein catabolism, positive regulation of proteolysis during cellular protein catabolic process, positive regulation of proteolysis during cellular protein catabolism, up regulation of peptidolysis during cellular protein catabolic process, up regulation of peptidolysis during cellular protein catabolism, up regulation of proteolysis during cellular protein catabolic process, up regulation of proteolysis during cellular protein catabolism, up-regulation of peptidolysis during cellular protein catabolic process, up-regulation of peptidolysis during cellular protein catabolism, up-regulation of proteolysis during cellular protein catabolic process, up-regulation of proteolysis during cellular protein catabolism, upregulation of peptidolysis during cellular protein catabolic process, upregulation of peptidolysis during cellular protein catabolism, upregulation of proteolysis during cellular protein catabolic process, upregulation of proteolysis during cellular protein catabolism Definition: Any process that activates or increases the frequency, rate or extent of proteolysis involved in protein catabolic process. Subtypes: positive regulation of proteolysis associated with antigen processing and presentation [GO:0002630], positive regulation of proteasomal protein catabolic process [GO:1901800], positive regulation of ubiquitin-dependent protein catabolic process [GO:2000060]